methyl-tetrahydromethanopterin:coenzyme M methyltransferase complex [GO:0044677] (cellular component) Relationships: is a type of GO:1902494 References: PMID:8477726 Sources: GOC:mengo_curators Definition: A protein complex consisted of eight polypeptides. This complex catalyzes the formation of methyl-coenzyme M and H4MPT from N5-methyl-H4MPT and CoM during methanogenesis. Also known as: coenzyme M methyltransferase complex, methyl-H4MPT, 5-methyl-5,6,7,8-tetrahydromethanopterin:2-mercaptoethane sulfonate 2-methyltransferase complex, N5-methyltetrahydromethanopterin-coenzyme M methyltransferase complex